regulation of hydrogen sulfide biosynthetic process [GO:1904826] (biological process) Also known as: regulation of hydrogen sulfide anabolism, regulation of hydrogen sulfide biosynthesis, regulation of hydrogen sulfide formation, regulation of hydrogen sulfide synthesis, regulation of hydrogen sulphide biosynthesis, regulation of hydrogen sulphide biosynthetic process Relationships: is a type of regulation of biosynthetic process [GO:0009889]; is a type of GO:0042762; regulates hydrogen sulfide biosynthetic process [GO:0070814] Subtypes: negative regulation of hydrogen sulfide biosynthetic process [GO:1904827], positive regulation of hydrogen sulfide biosynthetic process [GO:1904828] References: PMID:22034194 Sources: GOC:BHF, GOC:BHF_miRNA, GOC:TermGenie, GOC:rph, GO_REF:0000058 Definition: Any process that modulates the frequency, rate or extent of hydrogen sulfide biosynthetic process.